{
  "gene": "UniProtKB:P11169",
  "gene_symbol": "SLC2A3",
  "term_id": "GO:0070837",
  "term_label": "dehydroascorbic acid transport",
  "gene_name": "Solute carrier family 2, facilitated glucose transporter member 3"
}